{
  "gene": "UniProtKB:P13385",
  "gene_name": "Teratocarcinoma-derived growth factor 1",
  "gene_symbol": "TDGF1",
  "term_id": "GO:0005576",
  "term_label": "extracellular region"
}